1-undecene biosynthetic process [GO:1902821] (biological process) Also known as: 1-undecene anabolism, 1-undecene biosynthesis, 1-undecene formation, 1-undecene synthesis Definition: The chemical reactions and pathways resulting in the formation of 1-undecene. References: PMID:16013377 Sources: GOC:TermGenie, GOC:mengo_curators, GO_REF:0000068 Relationships: is a type of alkene biosynthetic process [GO:0043450]